[glycogen-synthase-D] phosphatase activity [GO:0050407] (molecular function) Definition: Catalysis of the reaction: [glycogen-synthase D] + H2O = [glycogen-synthase I] + phosphate. Also known as: Mg2+ dependent glycogen synthase phosphatase activity, UDP-glucose:glycogen 4-alpha-D-glucosyltransferase-D phosphohydrolase activity, UDP-glycogen glucosyltransferase phosphatase activity, UDPglucose-glycogen glucosyltransferase phosphatase activity, UDPglucose:glycogen 4-alpha-D-glucosyltransferase-D phosphohydrolase activity, glycogen glucosyltransferase phosphatase activity, glycogen synthase D phosphatase activity, glycogen synthase phosphatase activity, glycogen synthetase phosphatase activity, glycogen-synthase-D phosphatase activity, phosphatase type 2oC, uridine diphosphoglucose-glycogen glucosyltransferase phosphatase activity Sources: EC:3.1.3.42, MetaCyc:GLYCOGEN-SYNTHASE-D-PHOSPHATASE-RXN Relationships: is a type of phosphoprotein phosphatase activity [GO:0004721]